{
  "gene_symbol": "IGF2",
  "gene_name": "Insulin-like growth factor II",
  "term_label": "insulin-like growth factor receptor binding",
  "term_id": "GO:0005159",
  "gene": "UniProtKB:P01344"
}